{
  "gene_name": "Ciliary neurotrophic factor receptor subunit alpha",
  "gene": "UniProtKB:P26992",
  "gene_symbol": "CNTFR",
  "term_id": "GO:0009897",
  "term_label": "external side of plasma membrane"
}